{
  "gene": "UniProtKB:P30281",
  "term_label": "nucleus",
  "gene_symbol": "CCND3",
  "term_id": "GO:0005634",
  "gene_name": "G1_S-specific cyclin-D3"
}